{
  "gene": "UniProtKB:P15515",
  "term_id": "GO:0005615",
  "gene_symbol": "HTN1",
  "gene_name": "Histatin-1",
  "term_label": "extracellular space"
}